plus-end kinesin complex [GO:0005873] (cellular component) Sources: GOC:mah Relationships: is a type of kinesin complex [GO:0005871] Definition: Any complex that includes a dimer of molecules from the kinesin superfamily and any associated proteins, and moves towards the plus end of a microtubule.